{
  "term_label": "Unknown biological process",
  "gene_symbol": "PNRC1",
  "gene": "UniProtKB:Q12796",
  "gene_name": "Proline-rich nuclear receptor coactivator 1",
  "term_id": "UNKNOWN:0002"
}